pectic matrix [GO:0048217] (cellular component) Definition: The gel-like pectin matrix consists of the interlinked acidic and neutral pectin networks that are further cross-linked by calcium bridges. Pectins consist largely of long chains of mostly galacturonic acid units (typically 1,4 linkages and sometimes methyl esters). Three major pectic polysaccharides (homogalacturonan, rhamnogalacturonan I and rhamnogalacturonan II) are thought to occur in all primary cell walls. References: PMID:11554482 Sources: GOC:jid Relationships: is_a cellular anatomical structure [GO:0110165]; is part of primary cell wall [GO:0009530]; is part of secondary cell wall [GO:0009531]